{
  "term_id": "GO:0043235",
  "term_label": "receptor complex",
  "gene_symbol": "ABCG8",
  "gene": "UniProtKB:Q9H221",
  "gene_name": "ATP-binding cassette sub-family G member 8"
}